{
  "gene_symbol": "TNFSF11",
  "gene_name": "Tumor necrosis factor ligand superfamily member 11",
  "term_id": "GO:0005615",
  "gene": "UniProtKB:O14788",
  "term_label": "extracellular space"
}